cellular response to desipramine [GO:1904308] (biological process) References: PMID:20549303 Sources: GOC:TermGenie, GO_REF:0000071 Definition: Any process that results in a change in state or activity of a cell (in terms of movement, secretion, enzyme production, gene expression, etc.) as a result of a desipramine stimulus. Relationships: is_a cellular response to nitrogen compound [GO:1901699]; is a type of response to desipramine [GO:1904307]